icosatetraenoic acid binding [GO:0050543] (molecular function) Definition: Binding to icosatetraenoic acid, any straight-chain fatty acid with twenty carbon atoms and four double bonds per molecule. Also known as: eicosatetraenoic acid binding Subtypes: arachidonate binding [GO:0050544] Relationships: is a type of long-chain fatty acid binding [GO:0036041] Sources: ISBN:0198506732